{
  "term_id": "GO:0051895",
  "gene_name": "Integrin beta-1-binding protein 1",
  "gene": "UniProtKB:O14713",
  "term_label": "negative regulation of focal adhesion assembly",
  "gene_symbol": "ITGB1BP1"
}